{
  "term_id": "GO:1905413",
  "gene": "UniProtKB:O94812",
  "term_label": "regulation of dense core granule exocytosis",
  "gene_symbol": "BAIAP3",
  "gene_name": "BAI1-associated protein 3"
}